{
  "gene_name": "DDRGK domain-containing protein 1",
  "gene": "UniProtKB:Q96HY6",
  "term_label": "protein ufmylation",
  "term_id": "GO:0071569",
  "gene_symbol": "DDRGK1"
}